{
  "gene_name": "Kinase suppressor of Ras 2",
  "term_id": "GO:0005886",
  "term_label": "plasma membrane",
  "gene_symbol": "KSR2",
  "gene": "UniProtKB:Q6VAB6"
}